{
  "term_id": "GO:0005789",
  "gene_name": "Vacuolar ATPase assembly integral membrane protein VMA21",
  "gene": "UniProtKB:Q3ZAQ7",
  "term_label": "endoplasmic reticulum membrane",
  "gene_symbol": "VMA21"
}